{
  "term_id": "GO:0001228",
  "gene_symbol": "ZNF345",
  "term_label": "DNA-binding transcription activator activity, RNA polymerase II-specific",
  "gene_name": "Zinc finger protein 345",
  "gene": "UniProtKB:Q14585"
}